protein-tRNA adaptor activity [GO:0180014] (molecular function) References: PMID:31048492 Also known as: tRNA carrier Relationships: is a type of protein-RNA adaptor activity [GO:0140517] Definition: The binding activity of a protein that brings together another protein and a tRNA, permitting those molecules to function in a coordinated way.